{
  "term_id": "GO:0000467",
  "gene_symbol": "EXOSC2",
  "term_label": "exonucleolytic trimming to generate mature 3'-end of 5.8S rRNA from tricistronic rRNA transcript (SSU-rRNA, 5.8S rRNA, LSU-rRNA)",
  "gene_name": "Exosome complex component RRP4",
  "gene": "UniProtKB:Q13868"
}